{
  "gene": "UniProtKB:P0DMB1",
  "term_id": "UNKNOWN:0002",
  "gene_symbol": "PRR23D2",
  "term_label": "Unknown biological process",
  "gene_name": "Proline-rich protein 23D2"
}